{
  "gene_symbol": "CORO2B",
  "gene_name": "Coronin-2B",
  "term_label": "actin filament",
  "gene": "UniProtKB:Q9UQ03",
  "term_id": "GO:0005884"
}